dUMP biosynthetic process [GO:0006226] (biological process) Sources: ISBN:0198506732 Relationships: is a type of pyrimidine deoxyribonucleoside monophosphate biosynthetic process [GO:0009177]; is a type of pyrimidine deoxyribonucleotide biosynthetic process [GO:0009221]; is a type of GO:0046078 Also known as: dUMP anabolism, dUMP biosynthesis, dUMP formation, dUMP synthesis Definition: The chemical reactions and pathways resulting in the formation of dUMP, deoxyuridine monophosphate (2'-deoxyuridine 5'-phosphate).